{
  "term_label": "Cul4-RING E3 ubiquitin ligase complex",
  "gene_name": "DDB1- and CUL4-associated factor 16",
  "term_id": "GO:0080008",
  "gene": "UniProtKB:Q9NXF7",
  "gene_symbol": "DCAF16"
}